{
  "gene_name": "5-hydroxytryptamine receptor 3E",
  "gene_symbol": "HTR3E",
  "term_label": "chemical synaptic transmission",
  "gene": "UniProtKB:A5X5Y0",
  "term_id": "GO:0007268"
}